negative regulation of cell adhesion involved in single-species biofilm formation [GO:1900188] (biological process) Relationships: is a type of GO:0010812; is a type of GO:1900187; negatively regulates cell adhesion involved in single-species biofilm formation [GO:0043709] Sources: GOC:TermGenie, GOC:di Definition: Any process that stops, prevents or reduces the frequency, rate or extent of cell adhesion involved in single-species biofilm formation. Also known as: down regulation of cell adhesion involved in single-species biofilm formation, down-regulation of cell adhesion involved in single-species biofilm formation, downregulation of cell adhesion involved in single-species biofilm formation, inhibition of cell adhesion involved in single-species biofilm formation, down regulation of cell adhesion during single-species biofilm formation, down-regulation of cell adhesion during single-species biofilm formation, downregulation of cell adhesion during single-species biofilm formation, inhibition of cell adhesion during single-species biofilm formation, negative regulation of cell adhesion during single-species biofilm formation